{
  "gene": "UniProtKB:Q9UNH6",
  "term_id": "GO:0000407",
  "gene_name": "Sorting nexin-7",
  "gene_symbol": "SNX7",
  "term_label": "phagophore assembly site"
}